{
  "gene_name": "Zinc finger protein 410",
  "term_id": "GO:0003712",
  "gene_symbol": "ZNF410",
  "gene": "UniProtKB:Q86VK4",
  "term_label": "transcription coregulator activity"
}